regulation of protein localization to microtubule [GO:1902816] (biological process) Relationships: is a type of regulation of protein localization [GO:0032880]; regulates protein localization to microtubule [GO:0035372] Definition: Any process that modulates the frequency, rate or extent of protein localization to microtubule. Also known as: regulation of protein localisation to microtubule References: PMID:23087209 Sources: GOC:TermGenie, GOC:vw, GO_REF:0000058 Subtypes: GO:1902817